{
  "term_label": "chromosome condensation",
  "gene_symbol": "H1-7",
  "gene_name": "Testis-specific H1 histone",
  "term_id": "GO:0030261",
  "gene": "UniProtKB:Q75WM6"
}